{
  "term_id": "GO:0036376",
  "gene_symbol": "ATP1B2",
  "gene_name": "Sodium_potassium-transporting ATPase subunit beta-2",
  "gene": "UniProtKB:P14415",
  "term_label": "sodium ion export across plasma membrane"
}